synaptic vesicle budding [GO:0070142] (biological process) Definition: Evagination of a membrane to form a synaptic vesicle. Subtypes: synaptic vesicle budding from endosome [GO:0016182], synaptic vesicle budding from presynaptic endocytic zone membrane [GO:0016185] Sources: GOC:mah Relationships: is a type of vesicle budding from membrane [GO:0006900]; is part of synaptic vesicle transport [GO:0048489]